{
  "term_label": "Unknown cellular component",
  "gene_symbol": "ANKRD30B",
  "term_id": "UNKNOWN:0003",
  "gene": "UniProtKB:Q9BXX2",
  "gene_name": "Ankyrin repeat domain-containing protein 30B"
}